{
  "gene": "UniProtKB:Q8IYB4",
  "gene_name": "PEX5-related protein",
  "term_id": "GO:0005052",
  "gene_symbol": "PEX5L",
  "term_label": "peroxisome matrix targeting signal-1 binding"
}